{
  "gene_symbol": "SPTBN2",
  "term_id": "GO:0030036",
  "gene_name": "Spectrin beta chain, non-erythrocytic 2",
  "term_label": "actin cytoskeleton organization",
  "gene": "UniProtKB:O15020"
}